{
  "term_label": "G protein-coupled receptor activity",
  "gene_name": "Melatonin-related receptor",
  "term_id": "GO:0004930",
  "gene_symbol": "GPR50",
  "gene": "UniProtKB:Q13585"
}